{
  "term_label": "cytoplasm",
  "gene_name": "E3 ubiquitin-protein ligase CHIP",
  "gene": "UniProtKB:Q9UNE7",
  "term_id": "GO:0005737",
  "gene_symbol": "STUB1"
}